{
  "gene": "UniProtKB:P61026",
  "term_label": "exocytosis",
  "gene_name": "Ras-related protein Rab-10",
  "term_id": "GO:0006887",
  "gene_symbol": "RAB10"
}